detection of chemical stimulus involved in magnetoreception [GO:0050969] (biological process) Definition: The series of events involved in magnetoception in which a chemical stimulus is received and converted into a molecular signal. It is believed that organisms such as birds and salamanders interpret product ratios in chemical reactions which involve transitions between different spin states. Sources: GOC:ai, GOC:dos Also known as: magnetoception, sensory transduction of chemical stimulus, magnetoreception, detection of chemical stimulus, magnetoreception, sensory detection of chemical stimulus, magnetoreception, sensory transduction of chemical stimulus, sensory detection of chemical stimulus during magnetoreception, sensory transduction of chemical stimulus during magnetoreception Relationships: is a type of detection of chemical stimulus involved in sensory perception [GO:0050907]; BFO_0000050 magnetoreception by sensory perception of chemical stimulus [GO:0050977]